multivesicular body-lysosome fusion [GO:0061763] (biological process) Relationships: is a type of vesicle fusion [GO:0006906]; is a type of GO:0097212; BFO_0000050 endosome to lysosome transport via multivesicular body sorting pathway [GO:0032510] References: PMID:21118109 Sources: GOC:PARL, GOC:dph, GOC:pad Also known as: MVB-lysosome fusion, fusion of MVB to lysosome, fusion of multivesicular body to lysosome, endosome-lysosome fusion, late endosome-lysosome fusion Definition: The organelle membrane fusion process in which the membrane of a multivesicular body fuses with a lysosome to create a hybrid organelle.